{
  "term_id": "GO:0003682",
  "gene": "UniProtKB:Q6UXN9",
  "gene_symbol": "WDR82",
  "gene_name": "WD repeat-containing protein 82",
  "term_label": "chromatin binding"
}